{
  "term_label": "SMAD binding",
  "gene_symbol": "SKOR1",
  "term_id": "GO:0046332",
  "gene": "UniProtKB:P84550",
  "gene_name": "SKI family transcriptional corepressor 1"
}